3-ketoglucose-reductase activity [GO:0048258] (molecular function) Definition: Catalysis of the reaction: NADP+ + 3-dehydro-alpha-D-glucose = NADPH + alpha-D-glucose. Sources: MetaCyc:KETOGLUCOSE-REDUCTASE-RXN Relationships: is a type of oxidoreductase activity, acting on the CH-OH group of donors, NAD or NADP as acceptor [GO:0016616]